{
  "term_label": "GTPase activity",
  "term_id": "GO:0003924",
  "gene_symbol": "RASEF",
  "gene": "UniProtKB:Q8IZ41",
  "gene_name": "Ras and EF-hand domain-containing protein"
}